indole-2-monooxygenase activity [GO:0036190] (molecular function) Relationships: is a type of GO:0016712 Sources: RHEA:31899 Definition: Catalysis of the reaction: indole + O2 + reduced [NADPH--hemoprotein reductase] = H+ + H2O + indolin-2-one + oxidized [NADPH--hemoprotein reductase].